{
  "gene_symbol": "RBM28",
  "term_id": "UNKNOWN:0001",
  "gene": "UniProtKB:Q9NW13",
  "gene_name": "RNA-binding protein 28",
  "term_label": "Unknown molecular function"
}